{
  "term_id": "GO:0051724",
  "gene_name": "Peroxisomal membrane protein PMP34",
  "gene_symbol": "SLC25A17",
  "term_label": "NAD transmembrane transporter activity",
  "gene": "UniProtKB:O43808"
}